COPII vesicles tethering complex [GO:0106103] (cellular component) Relationships: is a type of GO:0098796; is a type of vesicle tethering complex [GO:0099023]; is part of cis-Golgi network membrane [GO:0033106] Also known as: GRASP65-GM130 complex, Bug1-Grh1 complex Definition: A protein complex that resides in the cis-golgi membrane and plays a role in the tethering of COPII vesicles, through an interaction with vesicle tethering proteins (p115 in H. Sapiens and Uso1 S. cerevisiae), granting the cis-Golgi and endoplasmic reticulum to Golgi vesicle-mediated transport. It is composed by GRASP65 and GM130 protein in H. sapiens and by Bug1 and Grh1 proteins in S. cerevisiae. References: PMID:21482742, PMID:9628863 Sources: GOC:lnp